{
  "gene_symbol": "CD81",
  "gene_name": "CD81 antigen",
  "term_id": "GO:0005886",
  "gene": "UniProtKB:P60033",
  "term_label": "plasma membrane"
}